hypersensitivity [GO:0002524] (biological process) Subtypes: type III hypersensitivity [GO:0001802], GO:0001806, GO:0002445, type I hypersensitivity [GO:0016068] Also known as: hypersensitivity response Sources: GOC:jal, ISBN:0781735149 Relationships: is a type of GO:0002438 Regulation: regulated by regulation of hypersensitivity [GO:0002883]; negatively regulated by negative regulation of hypersensitivity [GO:0002884]; positively regulated by GO:0002885 Definition: An inflammatory response to an exogenous environmental antigen or an endogenous antigen initiated by the adaptive immune system.